{
  "gene_symbol": "NEXN",
  "term_id": "GO:0005925",
  "gene_name": "Nexilin",
  "gene": "UniProtKB:Q0ZGT2",
  "term_label": "focal adhesion"
}